{
  "gene": "UniProtKB:Q07817",
  "gene_name": "Bcl-2-like protein 1",
  "term_id": "GO:0043065",
  "gene_symbol": "BCL2L1",
  "term_label": "positive regulation of apoptotic process"
}